{
  "gene_name": "Somatostatin receptor type 4",
  "gene": "UniProtKB:P31391",
  "term_id": "GO:0005886",
  "term_label": "plasma membrane",
  "gene_symbol": "SSTR4"
}